negative regulation of release of sequestered calcium ion into cytosol [GO:0051280] (biological process) Relationships: is a type of regulation of release of sequestered calcium ion into cytosol [GO:0051279]; is a type of positive regulation of sequestering of calcium ion [GO:0051284]; is a type of negative regulation of calcium ion transmembrane transport [GO:1903170]; negatively regulates release of sequestered calcium ion into cytosol [GO:0051209] Also known as: negative regulation of calcium ion (Ca2+) mobilization, negative regulation of calcium mobilization, negative regulation of cytoplasmic release of sequestered calcium ion (Ca2+), negative regulation of cytoplasmic release of stored calcium ion (Ca2+), negative regulation of release of sequestered calcium ion (Ca2+), negative regulation of release of sequestered calcium ion into cytoplasm, negative regulation of release of stored calcium ion (Ca2+), negative regulation of release of stored calcium ion (Ca2+) into cytoplasm, down regulation of release of sequestered calcium ion into cytosol, down-regulation of release of sequestered calcium ion into cytosol, downregulation of release of sequestered calcium ion into cytosol, negative regulation of cytosolic release of sequestered calcium ion (Ca2+), negative regulation of cytosolic release of stored calcium ion (Ca2+), negative regulation of release of stored calcium ion (Ca2+) into cytosol, inhibition of release of sequestered calcium ion into cytosol Sources: GOC:ai Definition: Any process that stops, prevents, or reduces the frequency, rate or extent of the release into the cytosolic compartment of calcium ions sequestered in the endoplasmic reticulum or mitochondria. Subtypes: negative regulation of ryanodine-sensitive calcium-release channel activity [GO:0060315]